{
  "gene_name": "Zinc finger imprinted 2",
  "term_id": "UNKNOWN:0001",
  "gene_symbol": "ZIM2",
  "gene": "UniProtKB:Q9NZV7",
  "term_label": "Unknown molecular function"
}